DNA-3-methylbase glycosylase activity [GO:0043733] (molecular function) Definition: Catalysis of the reaction: DNA containing 3-methylbase + H2O = DNA with abasic site + 3-methylbase. This reaction is the hydrolysis of DNA by cleavage of the N-C1' glycosidic bond between the damaged DNA 3-methylpurine or 3-methylpyrimidine base and the deoxyribose sugar to remove the methylated base, leaving an apurinic or apyrimidinic site. References: PMID:10777493, PMID:14517230 Relationships: is a type of GO:0003905 Subtypes: GO:0008725, GO:0052822 Also known as: Mag III, MagIII, DNA-3-methyladenine glycosylase III